{
  "gene": "UniProtKB:Q8NG81",
  "term_id": "GO:0004984",
  "gene_name": "Olfactory receptor 2M7",
  "term_label": "olfactory receptor activity",
  "gene_symbol": "OR2M7"
}